{
  "gene_name": "Tyrosine-protein phosphatase non-receptor type 2",
  "gene_symbol": "PTPN2",
  "term_id": "GO:0005737",
  "gene": "UniProtKB:P17706",
  "term_label": "cytoplasm"
}